{
  "term_label": "ether lipid biosynthetic process",
  "term_id": "GO:0008611",
  "gene": "UniProtKB:O15228",
  "gene_name": "Dihydroxyacetone phosphate acyltransferase",
  "gene_symbol": "GNPAT"
}